{
  "gene_symbol": "TXNDC12",
  "gene": "UniProtKB:O95881",
  "term_label": "endoplasmic reticulum",
  "gene_name": "Thioredoxin domain-containing protein 12",
  "term_id": "GO:0005783"
}